{
  "gene_name": "B-cell CLL_lymphoma 6 member B protein",
  "gene": "UniProtKB:Q8N143",
  "term_id": "GO:0045595",
  "gene_symbol": "BCL6B",
  "term_label": "regulation of cell differentiation"
}